{
  "term_id": "GO:0005794",
  "gene_symbol": "ARL1",
  "gene": "UniProtKB:P40616",
  "term_label": "Golgi apparatus",
  "gene_name": "ADP-ribosylation factor-like protein 1"
}